{
  "gene_name": "Autophagy protein 5",
  "gene": "UniProtKB:Q9H1Y0",
  "gene_symbol": "ATG5",
  "term_id": "GO:0061908",
  "term_label": "phagophore"
}